abducens nerve morphogenesis [GO:0021598] (biological process) Definition: The process in which the anatomical structure of the abducens nerve is generated and organized. The motor function of the abducens nerve is to contract the lateral rectus which results in abduction of the eye. Sources: GOC:cls, GOC:dgh, GOC:dph, GOC:jid, GO_REF:0000021 Relationships: is a type of GO:0021602; is part of abducens nerve development [GO:0021560] Also known as: CN VI development